{
  "gene_symbol": "OR5AK3P",
  "term_id": "GO:0004984",
  "gene": "UniProtKB:Q8NH89",
  "gene_name": "Putative olfactory receptor 5AK3",
  "term_label": "olfactory receptor activity"
}